{
  "gene_name": "E3 ubiquitin-protein ligase ZNF598",
  "term_id": "GO:0016567",
  "term_label": "protein ubiquitination",
  "gene_symbol": "ZNF598",
  "gene": "UniProtKB:Q86UK7"
}